{
  "term_label": "ammonium channel activity",
  "gene": "UniProtKB:P29972",
  "gene_symbol": "AQP1",
  "gene_name": "Aquaporin-1",
  "term_id": "GO:0008519"
}